{
  "term_label": "ubiquitin protein ligase activity",
  "gene_name": "E3 ubiquitin-protein ligase RFWD3",
  "gene_symbol": "RFWD3",
  "gene": "UniProtKB:Q6PCD5",
  "term_id": "GO:0061630"
}